{
  "term_label": "voltage-gated potassium channel complex",
  "gene_symbol": "KCNA7",
  "gene": "UniProtKB:Q96RP8",
  "term_id": "GO:0008076",
  "gene_name": "Potassium voltage-gated channel subfamily A member 7"
}